inositol trisphosphate kinase activity [GO:0051766] (molecular function) Relationships: is a type of phosphotransferase activity, alcohol group as acceptor [GO:0016773]; is a type of inositol phosphate kinase activity [GO:0180030] Sources: GOC:ai Also known as: IP3K Subtypes: inositol-1,4,5-trisphosphate 6-kinase activity [GO:0000823], inositol-1,4,5-trisphosphate 3-kinase activity [GO:0008440], inositol-1,3,4-trisphosphate 6-kinase activity [GO:0052725], inositol-1,3,4-trisphosphate 5-kinase activity [GO:0052726], GO:0052835 Definition: Catalysis of the reaction: inositol trisphosphate + ATP = inositol tetrakisphosphate + ADP + H+.